{
  "term_id": "GO:0048247",
  "gene_symbol": "SAA1",
  "gene": "UniProtKB:P0DJI8",
  "term_label": "lymphocyte chemotaxis",
  "gene_name": "Serum amyloid A-1 protein"
}